{
  "gene_name": "Leucine-rich repeat-containing G-protein coupled receptor 6",
  "term_id": "GO:0007411",
  "term_label": "axon guidance",
  "gene_symbol": "LGR6",
  "gene": "UniProtKB:Q9HBX8"
}